{
  "gene_name": "Tumor protein D55",
  "term_label": "Unknown biological process",
  "gene_symbol": "TPD52L3",
  "gene": "UniProtKB:Q96J77",
  "term_id": "UNKNOWN:0002"
}